cysteine dioxygenase activity [GO:0017172] (molecular function) Definition: Catalysis of the reaction: L-cysteine + O2 = 3-sulfino-L-alanine + H+. Relationships: is_a oxidoreductase activity, acting on single donors with incorporation of molecular oxygen, incorporation of two atoms of oxygen [GO:0016702] Sources: EC:1.13.11.20, RHEA:20441